dolichyl-phosphate-glucose-glycolipid alpha-glucosyltransferase activity [GO:0004583] (molecular function) Relationships: is a type of glucosyltransferase activity [GO:0046527] Sources: GOC:mah Subtypes: dolichyl pyrophosphate Man9GlcNAc2 alpha-1,3-glucosyltransferase activity [GO:0042281], GO:0042283, dolichyl pyrophosphate Glc2Man9GlcNAc2 alpha-1,2-glucosyltransferase activity [GO:0106073] Definition: Catalysis of the transfer of an alpha-D-glucosyl residue from dolichyl-phosphate D-glucose into a membrane lipid-linked oligosaccharide.